{
  "term_label": "RNA polymerase II transcription regulatory region sequence-specific DNA binding",
  "gene_name": "Zinc finger protein 101",
  "term_id": "GO:0000977",
  "gene": "UniProtKB:Q8IZC7",
  "gene_symbol": "ZNF101"
}